regulation of postsynaptic neurotransmitter receptor internalization [GO:0099149] (biological process) Definition: Any process that modulates the frequency, rate or extent of endocytosis of neurotransmitter receptor at the postsynapse. Sources: GOC:ai Also known as: regulation of postsynaptic neurotransmitter receptor endocytosis Relationships: is a type of regulation of receptor internalization [GO:0002090]; is_a regulation of biological quality [GO:0065008]; regulates postsynaptic neurotransmitter receptor internalization [GO:0098884]